{
  "term_id": "GO:0045159",
  "gene_name": "Lethal(2) giant larvae protein homolog 1",
  "gene": "UniProtKB:Q15334",
  "gene_symbol": "LLGL1",
  "term_label": "myosin II binding"
}